{
  "term_id": "UNKNOWN:0003",
  "gene_symbol": "CLCN6",
  "gene_name": "H(+)_Cl(-) exchange transporter 6",
  "term_label": "Unknown cellular component",
  "gene": "UniProtKB:P51797"
}